{
  "term_label": "plasma membrane",
  "term_id": "GO:0005886",
  "gene_name": "Low-density lipoprotein receptor-related protein 1B",
  "gene_symbol": "LRP1B",
  "gene": "UniProtKB:Q9NZR2"
}